{
  "term_id": "UNKNOWN:0001",
  "gene_name": "Uncharacterized protein C5orf67",
  "term_label": "Unknown molecular function",
  "gene_symbol": "C5orf67",
  "gene": "UniProtKB:F2Z3F1"
}